{
  "gene_name": "E3 ubiquitin-protein ligase NEDD4-like",
  "gene_symbol": "NEDD4L",
  "term_label": "receptor internalization",
  "gene": "UniProtKB:Q96PU5",
  "term_id": "GO:0031623"
}